regulation of cell cycle checkpoint [GO:1901976] (biological process) Subtypes: GO:0090231, negative regulation of cell cycle checkpoint [GO:1901977], positive regulation of cell cycle checkpoint [GO:1901978], regulation of DNA damage checkpoint [GO:2000001] Note: Note that this term should not be used for direct manual annotation as it should always be possible to specify the type of checkpoint (i.e mitotic spindle or DNA damage etc). Relationships: is a type of regulation of cell cycle phase transition [GO:1901987]; is a type of regulation of intracellular signal transduction [GO:1902531]; regulates cell cycle checkpoint signaling [GO:0000075] Also known as: regulation of G1/S checkpoint, regulation of G1/S transition checkpoint Definition: Any process that modulates the frequency, rate or extent of cell cycle checkpoint. References: PMID:23028116 Sources: GOC:TermGenie, GOC:mtg_cell_cycle